{
  "gene": "UniProtKB:A8MVX0",
  "gene_name": "Rho guanine nucleotide exchange factor 33",
  "gene_symbol": "ARHGEF33",
  "term_label": "Unknown molecular function",
  "term_id": "UNKNOWN:0001"
}